{
  "gene": "UniProtKB:Q9BSW2",
  "gene_symbol": "CRACR2A",
  "gene_name": "EF-hand calcium-binding domain-containing protein 4B",
  "term_label": "GTP binding",
  "term_id": "GO:0005525"
}